angiogenin-PRI complex [GO:0032311] (cellular component) Definition: A stable heterodimer of angiogenin and placental ribonuclease inhibitor; interaction between angiogenin and PRI prevents angiogenin binding to its receptor to stimulate angiogenesis. References: PMID:2706246, PMID:3470787 Also known as: angiogenin-placental ribonuclease inhibitor complex Relationships: is_a protein-containing complex [GO:0032991]; is part of extracellular region [GO:0005576]